{
  "gene_symbol": "PSMD9",
  "gene": "UniProtKB:O00233",
  "term_id": "GO:0070682",
  "gene_name": "26S proteasome non-ATPase regulatory subunit 9",
  "term_label": "proteasome regulatory particle assembly"
}